{
  "term_label": "synapse assembly",
  "term_id": "GO:0007416",
  "gene_name": "Adhesion G protein-coupled receptor L3",
  "gene_symbol": "ADGRL3",
  "gene": "UniProtKB:Q9HAR2"
}